{
  "gene": "UniProtKB:Q13488",
  "term_id": "GO:0005886",
  "gene_name": "V-type proton ATPase 116 kDa subunit a 3",
  "gene_symbol": "TCIRG1",
  "term_label": "plasma membrane"
}